{
  "term_label": "mitochondrial inner membrane",
  "gene": "UniProtKB:Q9Y2C4",
  "gene_symbol": "EXOG",
  "term_id": "GO:0005743",
  "gene_name": "Nuclease EXOG, mitochondrial"
}